nuclear migration to the embryo sac center [GO:0023003] (biological process) Also known as: nuclear migration to the embryo sac centre, nuclear migration to the female gametophyte center, nuclear migration to the female gametophyte centre, nuclear migration to the megagametophyte center, nuclear migration to the megagametophyte centre, nucleus migration to the female gametophyte center, nucleus migration to the female gametophyte centre Sources: GOC:jid, GOC:mtg_plant, ISBN:047186840X Definition: Migration of one of the four nuclei at each pole of the eight-nucleate embryo sac, to the center of the cell. Relationships: is a type of embryo sac nuclear migration [GO:0009562]